mesenchymal cell apoptotic process involved in mesonephric nephron morphogenesis [GO:1901146] (biological process) Sources: GOC:TermGenie, GOC:mtg_apoptosis Definition: Any mesenchymal cell apoptotic process that is involved in mesonephric nephron morphogenesis. Regulation: regulated by regulation of mesenchymal cell apoptotic process involved in mesonephric nephron morphogenesis [GO:0061295]; negatively regulated by negative regulation of mesenchymal cell apoptotic process involved in mesonephric nephron morphogenesis [GO:0061296]; positively regulated by GO:0061297 Relationships: is a type of GO:1901145; is part of mesonephric nephron morphogenesis [GO:0061228]